positive regulation of lipid catabolic process [GO:0050996] (biological process) Relationships: is a type of positive regulation of catabolic process [GO:0009896]; is a type of positive regulation of lipid metabolic process [GO:0045834]; is a type of regulation of lipid catabolic process [GO:0050994]; positively regulates lipid catabolic process [GO:0016042] Sources: GOC:ai Subtypes: positive regulation of triglyceride catabolic process [GO:0010898], positive regulation of glucocorticoid catabolic process [GO:0031951], GO:0032000, positive regulation of juvenile hormone catabolic process [GO:0045971], GO:0060697, positive regulation of palmitic acid catabolic process [GO:0106395], positive regulation of butyryl-CoA catabolic process to butanol [GO:1900499], positive regulation of butyryl-CoA catabolic process to butyrate [GO:1900502], positive regulation of prostaglandin catabolic process [GO:1905830], GO:2000753 Also known as: positive regulation of lipid breakdown, positive regulation of lipid catabolism, positive regulation of lipid degradation, up regulation of lipid catabolic process, up-regulation of lipid catabolic process, upregulation of lipid catabolic process, activation of lipid catabolic process, stimulation of lipid catabolic process Definition: Any process that activates or increases the frequency, rate or extent of the chemical reactions and pathways resulting in the breakdown of lipids.